{
  "gene_name": "Zinc finger protein 426",
  "gene": "UniProtKB:Q9BUY5",
  "gene_symbol": "ZNF426",
  "term_label": "regulation of transcription by RNA polymerase II",
  "term_id": "GO:0006357"
}